interleukin-10 production [GO:0032613] (biological process) Sources: GOC:mah Regulation: regulated by regulation of interleukin-10 production [GO:0032653]; negatively regulated by negative regulation of interleukin-10 production [GO:0032693]; positively regulated by GO:0032733 Also known as: IL-10 production, interleukin-10 biosynthetic process, interleukin-10 secretion Definition: The appearance of interleukin-10 due to biosynthesis or secretion following a cellular stimulus, resulting in an increase in its intracellular or extracellular levels. Relationships: is a type of cytokine production [GO:0001816]